RBL family protein binding [GO:0061675] (molecular function) References: PMID:22312473 Definition: Binding to a member of the rhamnose-binding lectin (RBL) family, a family of animal lectins that show specific binding activities to L-rhamnose or D-galactose. Relationships: is a type of protein binding [GO:0005515] Also known as: rhamnose-binding lectin family protein binding